indole-3-acetaldehyde reductase (NADPH) activity [GO:0047019] (MF) Definition: Catalysis of the reaction: indole-3-ethanol + NADP+ = (indol-3-yl)acetaldehyde + H+ + NADPH. Relationships: is a type of oxidoreductase activity, acting on the CH-OH group of donors, NAD or NADP as acceptor [GO:0016616] Also known as: (indol-3-yl)ethanol:NADP+ oxidoreductase activity, indole-3-ethanol:NADP+ oxidoreductase activity, indoleacetaldehyde (reduced nicotinamide adenine dinucleotide phosphate) reductase activity Sources: EC:1.1.1.191, RHEA:17037